oxidoreductase activity, acting on other nitrogenous compounds as donors, cytochrome as acceptor [GO:0016662] (molecular function) Relationships: is a type of oxidoreductase activity, acting on other nitrogenous compounds as donors [GO:0016661] Sources: EC:1.7.2.- Subtypes: GO:0016966, GO:0033740, nitrite reductase (cytochrome, ammonia-forming) activity [GO:0042279], GO:0050304, nitrite reductase (NO-forming) activity [GO:0050421], GO:0050626, hydrazine dehydrogenase activity [GO:0140287], hydrazine synthase activity [GO:0140304], hydroxylamine dehydrogenase activity [GO:0140305] Definition: Catalysis of an oxidation-reduction (redox) reaction in which a nitrogenous group, excluding NH and NH2 groups, acts as a hydrogen or electron donor and reduces a cytochrome.